plastid ADPG pyrophosphorylase complex [GO:0031009] (cellular component) Subtypes: GO:0030932, chloroplast ADPG pyrophosphorylase complex [GO:0030933] Relationships: is a type of GO:0030931; is part of plastid [GO:0009536] Definition: An ADPG pyrophosphorylase complex found in a plastid. Sources: GOC:mah